endothelin maturation [GO:0034959] (biological process) Sources: GOC:BHF, GOC:rl Relationships: is a type of peptide hormone processing [GO:0016486]; is part of regulation of systemic arterial blood pressure by endothelin [GO:0003100] Definition: The process leading to the attainment of the full functional capacity of endothelin by conversion of Big-endothelin substrate into mature endothelin.